{
  "term_label": "GINS complex",
  "gene": "UniProtKB:Q14691",
  "term_id": "GO:0000811",
  "gene_name": "DNA replication complex GINS protein PSF1",
  "gene_symbol": "GINS1"
}